{
  "term_id": "GO:0007018",
  "gene": "UniProtKB:Q9UIL4",
  "term_label": "microtubule-based movement",
  "gene_symbol": "KIF25",
  "gene_name": "Kinesin-like protein KIF25"
}